{
  "gene_name": "Beta-parvin",
  "gene": "UniProtKB:Q9HBI1",
  "term_label": "actin cytoskeleton organization",
  "term_id": "GO:0030036",
  "gene_symbol": "PARVB"
}